{
  "gene_symbol": "CELF1",
  "term_label": "nucleus",
  "gene_name": "CUGBP Elav-like family member 1",
  "gene": "UniProtKB:Q92879",
  "term_id": "GO:0005634"
}